cilium assembly [GO:0060271] (biological process) Relationships: is a type of GO:0044782; is a type of organelle assembly [GO:0070925]; is a type of plasma membrane bounded cell projection assembly [GO:0120031]; has part axoneme assembly [GO:0035082]; has part intraciliary transport involved in cilium assembly [GO:0035735]; has part protein localization to cilium [GO:0061512]; has part ciliary basal body-plasma membrane docking [GO:0097711]; has part vesicle targeting, trans-Golgi to periciliary membrane compartment [GO:0097712]; has part GO:1905349 References: PMID:13978319, PMID:27350441 Sources: GOC:BHF, GOC:cilia, GOC:dph, GOC:kmv, GOC:pr Subtypes: motile cilium assembly [GO:0044458], GO:0061824, GO:1905515 Note: Note that we deem cilium and microtubule-based flagellum to be equivalent. Definition: The assembly of a cilium, a specialized eukaryotic organelle that consists of a filiform extrusion of the cell surface. Each cilium is bounded by an extrusion of the cytoplasmic membrane, and contains a regular longitudinal array of microtubules, anchored basally in a centriole. Also known as: ciliogenesis, cilium formation, microtubule-based flagellum assembly, cilium biogenesis, cilium morphogenesis, cilium organization Regulation: positively regulated by positive regulation of cilium assembly [GO:0045724]; regulated by regulation of cilium assembly [GO:1902017]; negatively regulated by GO:1902018